histone H3 ubiquitin ligase activity [GO:0141055] (molecular function) Subtypes: histone H3K23 ubiquitin ligase activity [GO:0140234], histone H3K18 ubiquitin ligase activity [GO:0140248], histone H3K14 ubiquitin ligase activity [GO:0140851] References: PMID:25303536 Relationships: is a type of histone ubiquitin ligase activity [GO:0140852] Definition: Catalysis of the transfer of ubiquitin to a histone H3 substrate.